{
  "gene_symbol": "ECHDC2",
  "term_id": "GO:0006635",
  "gene_name": "Enoyl-CoA hydratase domain-containing protein 2, mitochondrial",
  "gene": "UniProtKB:Q86YB7",
  "term_label": "fatty acid beta-oxidation"
}